citramalate CoA-transferase activity [GO:0047775] (molecular function) Also known as: acetyl-CoA:citramalate CoA-transferase activity Definition: Catalysis of the reaction: acetyl-CoA + citramalate = acetate + (3S)-citramalyl-CoA. Sources: EC:2.8.3.11, MetaCyc:CITRAMALATE-COA-TRANSFERASE-RXN Relationships: is a type of CoA-transferase activity [GO:0008410]